{
  "gene": "UniProtKB:P07203",
  "term_label": "mitochondrion",
  "gene_symbol": "GPX1",
  "term_id": "GO:0005739",
  "gene_name": "Glutathione peroxidase 1"
}